{
  "gene_name": "Inositol-trisphosphate 3-kinase B",
  "term_id": "GO:0032958",
  "term_label": "inositol phosphate biosynthetic process",
  "gene_symbol": "ITPKB",
  "gene": "UniProtKB:P27987"
}